regulation of GABA-A receptor activity [GO:0106040] (biological process) Relationships: is a type of regulation of signaling receptor activity [GO:0010469]; regulates GABA-A receptor activity [GO:0004890] Definition: Any process that modulates the frequency, rate or extent of GABA-A receptor activity. References: PMID:24044036